{
  "term_id": "GO:0000974",
  "gene_name": "Pre-mRNA-splicing factor SYF1",
  "gene": "UniProtKB:Q9HCS7",
  "gene_symbol": "XAB2",
  "term_label": "Prp19 complex"
}